{
  "gene": "UniProtKB:O75128",
  "gene_symbol": "COBL",
  "gene_name": "Protein cordon-bleu",
  "term_label": "actin filament network formation",
  "term_id": "GO:0051639"
}